{
  "gene_symbol": "HDGFL2",
  "term_label": "nucleus",
  "gene": "UniProtKB:Q7Z4V5",
  "term_id": "GO:0005634",
  "gene_name": "Hepatoma-derived growth factor-related protein 2"
}